{
  "gene_name": "Lipid transferase CIDEC",
  "term_label": "apoptotic process",
  "gene": "UniProtKB:Q96AQ7",
  "term_id": "GO:0006915",
  "gene_symbol": "CIDEC"
}